{
  "term_label": "plasma membrane",
  "gene": "UniProtKB:P54849",
  "term_id": "GO:0005886",
  "gene_symbol": "EMP1",
  "gene_name": "Epithelial membrane protein 1"
}